{
  "gene_name": "UMP-CMP kinase",
  "gene": "UniProtKB:P30085",
  "gene_symbol": "CMPK1",
  "term_id": "GO:0005737",
  "term_label": "cytoplasm"
}